{
  "term_id": "GO:0005886",
  "gene_symbol": "RAPH1",
  "term_label": "plasma membrane",
  "gene_name": "Ras-associated and pleckstrin homology domains-containing protein 1",
  "gene": "UniProtKB:Q70E73"
}